{
  "term_id": "GO:0006667",
  "term_label": "sphinganine metabolic process",
  "gene": "UniProtKB:Q6QHC5",
  "gene_symbol": "DEGS2",
  "gene_name": "Sphingolipid delta(4)-desaturase_C4-monooxygenase DES2"
}